{
  "gene": "UniProtKB:Q9NQ29",
  "gene_symbol": "LUC7L",
  "term_label": "mRNA binding",
  "term_id": "GO:0003729",
  "gene_name": "Putative RNA-binding protein Luc7-like 1"
}